{
  "term_id": "GO:0006357",
  "gene_name": "Zinc finger protein 529",
  "gene_symbol": "ZNF529",
  "gene": "UniProtKB:Q6P280",
  "term_label": "regulation of transcription by RNA polymerase II"
}